{
  "term_label": "receptor ligand activity",
  "gene_symbol": "IGFBP7",
  "gene_name": "Insulin-like growth factor-binding protein 7",
  "gene": "UniProtKB:Q16270",
  "term_id": "GO:0048018"
}